{
  "gene": "UniProtKB:Q9BTD3",
  "term_id": "UNKNOWN:0002",
  "gene_name": "Transmembrane protein 121",
  "gene_symbol": "TMEM121",
  "term_label": "Unknown biological process"
}